{
  "gene_symbol": "NEUROD1",
  "term_id": "GO:0045944",
  "gene_name": "Neurogenic differentiation factor 1",
  "term_label": "positive regulation of transcription by RNA polymerase II",
  "gene": "UniProtKB:Q13562"
}